{
  "gene_symbol": "SEMA7A",
  "gene_name": "Semaphorin-7A",
  "term_label": "semaphorin-plexin signaling pathway",
  "term_id": "GO:0071526",
  "gene": "UniProtKB:O75326"
}